{
  "term_id": "GO:0070292",
  "term_label": "N-acylphosphatidylethanolamine metabolic process",
  "gene": "UniProtKB:Q6IQ20",
  "gene_name": "N-acyl-phosphatidylethanolamine-hydrolyzing phospholipase D",
  "gene_symbol": "NAPEPLD"
}